alpha-1,6-mannosylglycoprotein 2-beta-N-acetylglucosaminyltransferase activity [GO:0008455] (molecular function) Sources: EC:2.4.1.143 Definition: Catalysis of the reaction: UDP-N-acetyl-D-glucosamine + alpha-D-mannosyl-1,6-(N-acetyl-beta-D-glucosaminyl-1,2-alpha-D-mannosyl-1,3)-beta-D-mannosyl-R = UDP + N-acetyl-beta-D-glucosaminyl-1,2-alpha-D-mannosyl-1,6-(N-acetyl-beta-D-glucosaminyl-1,2-alpha-D-mannosyl-1,3)-beta-D-mannosyl-R. Also known as: alpha-1,6-mannosylglycoprotein beta-1,2-N-acetylglucosaminyltransferase activity, GnTII activity, N-acetylglucosaminyltransferase II activity, N-glycosyl-oligosaccharide-glycoprotein N-acetylglucosaminyltransferase II activity, UDP-GlcNAc:mannoside alpha-(1,6) acetylglucosaminyltransferase activity, UDP-GlcNAc:mannoside alpha-1,6 acetylglucosaminyltransferase activity, UDP-N-acetyl-D-glucosamine:6-(alpha-D-mannosyl)-beta-D-mannosyl-glycoprotein 2-beta-N-acetyl-D-glucosaminyltransferase activity, acetylglucosaminyltransferase II activity, alpha-1,6-mannosyl-glycoprotein 2-beta-N-acetylglucosaminyltransferase activity, alpha-1,6-mannosyl-glycoprotein beta-1,2-N-acetylglucosaminyltransferase activity, uridine diphosphoacetylglucosamine-alpha-1,6-mannosylglycoprotein beta-1,2-N-acetylglucosaminyltransferase activity, uridine diphosphoacetylglucosamine-alpha-D-mannoside beta(1,2)-acetylglucosaminyltransferase activity, uridine diphosphoacetylglucosamine-alpha-D-mannoside beta-1,2-acetylglucosaminyltransferase activity, uridine diphosphoacetylglucosamine-mannoside alpha(1,6)-acetylglucosaminyltransferase activity, uridine diphosphoacetylglucosamine-mannoside alpha-1,6-acetylglucosaminyltransferase activity Relationships: is a type of acetylglucosaminyltransferase activity [GO:0008375]; is a type of catalytic activity, acting on a glycoprotein [GO:0140103]